mesenchymal stem cell maintenance involved in nephron morphogenesis [GO:0072038] (biological process) Subtypes: mesenchymal stem cell maintenance involved in mesonephric nephron morphogenesis [GO:0061235], mesenchymal stem cell maintenance involved in metanephric nephron morphogenesis [GO:0072309] Sources: GOC:mtg_kidney_jan10 Relationships: is a type of somatic stem cell population maintenance [GO:0035019]; is part of GO:0072028 Definition: The process in which an organism retains a population of mesenchymal stem cells that contributes to the shaping of a nephron. A mesenchymal stem cell is a cell that retains the ability to divide and proliferate throughout life to provide progenitor cells that can differentiate into specialized mesenchymal cells. Regulation: regulated by regulation of mesenchymal cell apoptotic process involved in nephron morphogenesis [GO:0072039]; negatively regulated by GO:0072040; positively regulated by GO:0072041